{
  "term_label": "cytosol",
  "gene_name": "Serine_threonine-protein kinase RIO2",
  "gene_symbol": "RIOK2",
  "gene": "UniProtKB:Q9BVS4",
  "term_id": "GO:0005829"
}